{
  "term_id": "GO:0061630",
  "gene": "UniProtKB:Q96PX1",
  "gene_symbol": "RNF157",
  "gene_name": "E3 ubiquitin ligase RNF157",
  "term_label": "ubiquitin protein ligase activity"
}